{
  "term_label": "Unknown cellular component",
  "gene_symbol": "ASB13",
  "term_id": "UNKNOWN:0003",
  "gene": "UniProtKB:Q8WXK3",
  "gene_name": "Ankyrin repeat and SOCS box protein 13"
}